{
  "gene_symbol": "APH1B",
  "term_id": "GO:0034205",
  "gene_name": "Gamma-secretase subunit APH-1B",
  "gene": "UniProtKB:Q8WW43",
  "term_label": "amyloid-beta formation"
}